cell adhesion involved in sprouting angiogenesis [GO:0120078] (biological process) Definition: The attachment of a cell, either to another cell or to an underlying substrate such as the extracellular matrix, via cell adhesion molecules that contributes to the formation of a blood vessel network. References: PMID:28264837 Sources: GOC:cvs Also known as: cell adhesion involved in blood vessel anastomosis, cell adhesion involved in vascular anastomosis Relationships: is a type of GO:0007155; is part of angiogenic sprout fusion [GO:0120077] Regulation: regulated by GO:0106088; negatively regulated by GO:0106089; positively regulated by GO:0106090